negative regulation of lymphocyte proliferation [GO:0050672] (biological process) Definition: Any process that stops, prevents or reduces the rate or extent of lymphocyte proliferation. Relationships: is a type of negative regulation of mononuclear cell proliferation [GO:0032945]; is a type of regulation of lymphocyte proliferation [GO:0050670]; is a type of negative regulation of lymphocyte activation [GO:0051250]; negatively regulates lymphocyte proliferation [GO:0046651] Also known as: down regulation of lymphocyte proliferation, down-regulation of lymphocyte proliferation, downregulation of lymphocyte proliferation, inhibition of lymphocyte proliferation Subtypes: negative regulation of B cell proliferation [GO:0030889], negative regulation of natural killer cell proliferation [GO:0032818], negative regulation of T cell proliferation [GO:0042130] Sources: GOC:ai